{
  "gene": "UniProtKB:Q96P48",
  "gene_symbol": "ARAP1",
  "term_label": "phosphatidylinositol-3,4,5-trisphosphate binding",
  "gene_name": "Arf-GAP with Rho-GAP domain, ANK repeat and PH domain-containing protein 1",
  "term_id": "GO:0005547"
}